{
  "term_label": "cytosol",
  "term_id": "GO:0005829",
  "gene_name": "Methylosome subunit pICln",
  "gene_symbol": "CLNS1A",
  "gene": "UniProtKB:P54105"
}